nuclear matrix anchoring at nuclear membrane [GO:0090292] (biological process) Definition: The process in which the nuclear matrix, the dense fibrillar network lying on the inner side of the nuclear membrane, is directly or indirectly linked to the nuclear membrane. Also known as: nucleoskeleton anchoring at nuclear membrane Relationships: is a type of nuclear matrix organization [GO:0043578]; is a type of maintenance of protein location in nucleus [GO:0051457] Sources: GOC:tb